gamma-aminobutyric acid receptor clustering [GO:0097112] (biological process) Also known as: GABA receptor clustering References: PMID:15620359 Sources: GOC:BHF, GOC:sjp Definition: The receptor clustering process in which gamma-aminobutyric acid (GABA) receptors are localized to distinct domains in the cell membrane. Relationships: is a type of GO:0072578; is part of GO:0001941